regulation of bone mineralization [GO:0030500] (biological process) Relationships: is a type of regulation of ossification [GO:0030278]; is_a regulation of biomineral tissue development [GO:0070167]; RO_0002211 bone mineralization [GO:0030282] Subtypes: positive regulation of bone mineralization [GO:0030501], negative regulation of bone mineralization [GO:0030502], regulation of bone mineralization involved in bone maturation [GO:1900157] Definition: Any process that modulates the frequency, rate or extent of bone mineralization. Sources: GOC:go_curators